regulation of BMP secretion [GO:2001284] (biological process) Sources: GOC:sart Subtypes: positive regulation of BMP secretion [GO:1900144], negative regulation of BMP secretion [GO:2001285] Also known as: regulation of BMP protein secretion, regulation of bone morphogenetic protein secretion Definition: Any process that modulates the frequency, rate or extent of BMP secretion. Relationships: is a type of GO:0010646; is a type of regulation of signaling [GO:0023051]; is a type of regulation of protein secretion [GO:0050708]; regulates BMP secretion [GO:0038055]